{
  "gene_symbol": "C6orf132",
  "gene": "UniProtKB:Q5T0Z8",
  "gene_name": "Uncharacterized protein C6orf132",
  "term_id": "UNKNOWN:0002",
  "term_label": "Unknown biological process"
}